{
  "term_id": "GO:0003712",
  "gene_symbol": "PBXIP1",
  "term_label": "transcription coregulator activity",
  "gene": "UniProtKB:Q96AQ6",
  "gene_name": "Pre-B-cell leukemia transcription factor-interacting protein 1"
}